{
  "term_id": "GO:0017022",
  "gene": "UniProtKB:P68032",
  "gene_symbol": "ACTC1",
  "gene_name": "Actin, alpha cardiac muscle 1",
  "term_label": "myosin binding"
}